{
  "gene": "UniProtKB:Q9GZP1",
  "term_id": "GO:0007399",
  "term_label": "nervous system development",
  "gene_name": "Neurensin-2",
  "gene_symbol": "NRSN2"
}